{
  "term_id": "UNKNOWN:0002",
  "term_label": "Unknown biological process",
  "gene_symbol": "PRR20G",
  "gene_name": "Proline-rich protein 20G",
  "gene": "UniProtKB:P0DPQ3"
}